{
  "gene_name": "MBT domain-containing protein 1",
  "term_label": "negative regulation of DNA-templated transcription",
  "term_id": "GO:0045892",
  "gene_symbol": "MBTD1",
  "gene": "UniProtKB:Q05BQ5"
}